pheophytinase activity [GO:0080124] (molecular function) Definition: Catalysis of the reaction: pheophytin + H2O = phytol + pheophorbide. References: PMID:19304936 Also known as: pheophytin pheophorbide hydrolase activity Relationships: is a type of carboxylic ester hydrolase activity [GO:0052689]